folic acid-containing compound biosynthetic process [GO:0009396] (biological process) Definition: The chemical reactions and pathways resulting in the formation of folic acid and its derivatives. Sources: GOC:ai Also known as: folate and derivative biosynthesis, folate and derivative biosynthetic process, folate-containing compound biosynthesis, folate-containing compound biosynthetic process, folic acid and derivative biosynthesis, folic acid and derivative biosynthetic process, folic acid-containing compound anabolism, folic acid-containing compound biosynthesis, folic acid-containing compound formation, folic acid-containing compound synthesis, vitamin B9 and derivative biosynthesis, vitamin B9 and derivative biosynthetic process, vitamin M and derivative biosynthesis, vitamin M and derivative biosynthetic process Subtypes: dihydrofolate biosynthetic process [GO:0006761], tetrahydrofolate biosynthetic process [GO:0046654], folic acid biosynthetic process [GO:0046656], tetrahydrofolylpolyglutamate biosynthetic process [GO:0046901] Relationships: is a type of folic acid-containing compound metabolic process [GO:0006760]; is a type of modified amino acid biosynthetic process [GO:0042398]; is a type of pteridine-containing compound biosynthetic process [GO:0042559]